spindle pole body organization [GO:0051300] (biological process) Subtypes: GO:0030474, GO:1905047, GO:1990395 Sources: GOC:ai, GOC:dph, GOC:jl, GOC:mah Relationships: is a type of cell cycle process [GO:0022402]; is a type of microtubule organizing center organization [GO:0031023] Also known as: SPB organization, spindle pole body organisation, SPB maturation, spindle pole body maturation, spindle pole body organization and biogenesis Definition: A process that is carried out at the cellular level which results in the assembly, arrangement of constituent parts, or disassembly of the spindle pole body (SPB). The SPB is the microtubule organizing center in fungi, and is functionally homologous to the animal cell centrosome.